{
  "term_label": "neuron projection",
  "gene": "UniProtKB:Q9Y2J0",
  "gene_name": "Rabphilin-3A",
  "term_id": "GO:0043005",
  "gene_symbol": "RPH3A"
}